cellular response to L-glutamine [GO:1904845] (biological process) Definition: Any process that results in a change in state or activity of a cell (in terms of movement, secretion, enzyme production, gene expression, etc.) as a result of a L-glutamine stimulus. References: PMID:23185570 Sources: GOC:TermGenie, GO_REF:0000071 Relationships: is a type of cellular response to amino acid stimulus [GO:0071230]; is a type of GO:1901699; is a type of cellular response to oxygen-containing compound [GO:1901701]; is a type of GO:1904844